mating projection septin ring [GO:0032175] (cellular component) Relationships: is a type of septin ring [GO:0005940]; is part of mating projection [GO:0005937] Definition: A septin ring, i.e. a ring-shaped structure composed of septins and septin-associated proteins, located at the neck of a shmoo (mating projection). The septin ring in the neck of a shmoo may act as a barrier to localize mating factors in the shmoo tip. References: PMID:16151244 Sources: GOC:krc, GOC:mah